{
  "term_label": "heterotypic cell-cell adhesion",
  "gene_symbol": "CD200",
  "term_id": "GO:0034113",
  "gene_name": "OX-2 membrane glycoprotein",
  "gene": "UniProtKB:P41217"
}